venom-mediated dermonecrosis in another organism [GO:0141123] (biological process) Definition: The disruption of the skin of another organism, leading to damage or temporary subversion of the skin. References: PMID:28194160 Relationships: is a type of venom-mediated disruption of anatomical structure in another organism [GO:0140138]